{
  "term_label": "positive regulation of cell migration",
  "gene_name": "Semaphorin-4A",
  "term_id": "GO:0030335",
  "gene_symbol": "SEMA4A",
  "gene": "UniProtKB:Q9H3S1"
}